neuromedin U receptor activity [GO:0001607] (molecular function) Definition: Combining with neuromedin U to initiate a change in cell activity. Sources: GOC:ai Also known as: NMUR activity Relationships: is a type of neuropeptide receptor activity [GO:0008188]; has part neuromedin U binding [GO:0042924]